{
  "term_label": "nucleus",
  "gene_name": "Importin subunit alpha-8",
  "gene": "UniProtKB:A9QM74",
  "gene_symbol": "KPNA7",
  "term_id": "GO:0005634"
}